{
  "gene_symbol": "HOXD12",
  "term_id": "UNKNOWN:0002",
  "gene": "UniProtKB:P35452",
  "term_label": "Unknown biological process",
  "gene_name": "Homeobox protein Hox-D12"
}